{
  "term_label": "Unknown molecular function",
  "gene": "UniProtKB:O95257",
  "term_id": "UNKNOWN:0001",
  "gene_name": "Growth arrest and DNA damage-inducible protein GADD45 gamma",
  "gene_symbol": "GADD45G"
}